{
  "term_id": "GO:0006654",
  "gene_symbol": "AGPAT2",
  "gene_name": "1-acyl-sn-glycerol-3-phosphate acyltransferase beta",
  "gene": "UniProtKB:O15120",
  "term_label": "phosphatidic acid biosynthetic process"
}